{
  "term_label": "membrane",
  "gene_symbol": "VSTM2A",
  "gene_name": "V-set and transmembrane domain-containing protein 2A",
  "gene": "UniProtKB:Q8TAG5",
  "term_id": "GO:0016020"
}